ammonia monooxygenase activity [GO:0018597] (molecular function) Definition: Catalysis of the reaction: AH2 + NH4+ + O2 = A + H+ + H2O + hydroxylamine. Relationships: is a type of GO:0004497; is_a oxidoreductase activity, acting on paired donors, with incorporation or reduction of molecular oxygen [GO:0016705] References: PMID:16347810 Sources: RHEA:27341